transcription factor TFIIH holo complex binding [GO:0062058] (molecular function) Relationships: is a type of protein-containing complex binding [GO:0044877] Definition: Binding to a transcription factor TFIIH holo complex. References: PMID:11259578